{
  "term_label": "nucleus",
  "term_id": "GO:0005634",
  "gene": "UniProtKB:Q10570",
  "gene_name": "Cleavage and polyadenylation specificity factor subunit 1",
  "gene_symbol": "CPSF1"
}